{
  "gene_name": "Regulator of G-protein signaling 9",
  "term_label": "GTPase activator activity",
  "term_id": "GO:0005096",
  "gene": "UniProtKB:O75916",
  "gene_symbol": "RGS9"
}